Atg12 ligase activity [GO:0061660] (molecular function) Definition: Catalysis of the transfer of Atg12 to a substrate protein via the reaction X-Atg12 + S = X + S-Atg12, where X is either an E2 or E3 enzyme, the X-Atg12 linkage is a thioester bond, and the S-Atg12 linkage is an isopeptide bond between the C-terminal amino acid of Atg12 and the epsilon-amino group of lysine residues in the substrate. Sources: GOC:dph Also known as: E3 Relationships: is a type of Atg12 transferase activity [GO:0019777]; is a type of ubiquitin-like protein ligase activity [GO:0061659]